positive regulation of beta 2 integrin biosynthetic process [GO:0045775] (biological process) Also known as: positive regulation of beta 2 integrin anabolism, positive regulation of beta 2 integrin biosynthesis, positive regulation of beta 2 integrin formation, positive regulation of beta 2 integrin synthesis, up regulation of beta 2 integrin biosynthetic process, up-regulation of beta 2 integrin biosynthetic process, upregulation of beta 2 integrin biosynthetic process, activation of beta 2 integrin biosynthetic process, stimulation of beta 2 integrin biosynthetic process Definition: Any process that activates or increases the frequency, rate or extent of the chemical reactions and pathways resulting in the formation of beta 2 integrins. Sources: GOC:go_curators Relationships: is a type of regulation of beta 2 integrin biosynthetic process [GO:0045115]; is a type of positive regulation of integrin biosynthetic process [GO:0045726]; positively regulates beta 2 integrin biosynthetic process [GO:0045114]